{
  "gene": "UniProtKB:Q8IXQ6",
  "term_label": "negative regulation of gene expression",
  "gene_name": "Protein mono-ADP-ribosyltransferase PARP9",
  "gene_symbol": "PARP9",
  "term_id": "GO:0010629"
}